{
  "gene_name": "Cyclin-dependent kinase 6",
  "gene": "UniProtKB:Q00534",
  "gene_symbol": "CDK6",
  "term_id": "GO:0005737",
  "term_label": "cytoplasm"
}